{
  "term_label": "Unknown biological process",
  "term_id": "UNKNOWN:0002",
  "gene": "UniProtKB:Q7RTR8",
  "gene_symbol": "TAS2R42",
  "gene_name": "Taste receptor type 2 member 42"
}